{
  "gene_symbol": "DYDC2",
  "term_label": "axoneme",
  "term_id": "GO:0005930",
  "gene": "UniProtKB:Q96IM9",
  "gene_name": "DPY30 domain-containing protein 2"
}